L-seryl-tRNA(Sec) kinase activity [GO:0043915] (molecular function) Also known as: O-phosphoseryl-tRNA(Sec) kinase activity Definition: Catalysis of the reaction: ATP + L-seryl-tRNA(Sec) = ADP + O-phospho-L-seryl-tRNA(Sec). Relationships: is a type of kinase activity [GO:0016301]; is a type of GO:0016773; is a type of catalytic activity, acting on a tRNA [GO:0140101] References: PMID:16201757 Sources: GOC:jl, RHEA:25037